{
  "gene": "UniProtKB:Q86V59",
  "gene_symbol": "PNMA8A",
  "gene_name": "Paraneoplastic antigen-like protein 8A",
  "term_label": "Unknown cellular component",
  "term_id": "UNKNOWN:0003"
}